tyramine biosynthetic process [GO:1901695] (biological process) Definition: The chemical reactions and pathways resulting in the formation of tyramine. Relationships: is a type of GO:0046189; is a type of primary amino compound biosynthetic process [GO:1901162] Also known as: tyramine anabolism, tyramine biosynthesis, tyramine formation, tyramine synthesis References: PMID:21284755 Sources: GOC:TermGenie